{
  "term_id": "GO:0033263",
  "term_label": "CORVET complex",
  "gene_name": "Transforming growth factor-beta receptor-associated protein 1",
  "gene_symbol": "TGFBRAP1",
  "gene": "UniProtKB:Q8WUH2"
}